{
  "gene_name": "Double homeobox protein 4-like protein 5",
  "term_label": "regulation of transcription by RNA polymerase II",
  "gene_symbol": "DUX4L5",
  "gene": "UniProtKB:P0CJ88",
  "term_id": "GO:0006357"
}